{
  "term_id": "GO:0005634",
  "gene_symbol": "ZNF112",
  "term_label": "nucleus",
  "gene": "UniProtKB:Q9UJU3",
  "gene_name": "Zinc finger protein 112"
}